acyl-lipid Delta(12)-acetylenase [GO:0016720] (molecular function) Definition: Catalysis of the reaction: (9Z,12Z)-octadecadienoyl-containing glycerolipid + 2 Fe(II)-[cytochrome b5] + 2 H+ + O2 = a (9Z)-octadec-9-en-12-ynoyl-containing glycerolipid + 2 Fe(III)-[cytochrome b5] + 2 H2O. Sources: RHEA:46552 Also known as: D12-fatty acid dehydrogenase activity, Delta12 fatty acid acetylenase, linoleate delta-12-fatty acid acetylenase (desaturase) activity, delta12-fatty acid dehydrogenase activity Relationships: is a type of oxidoreductase activity, acting on paired donors, with oxidation of a pair of donors resulting in the reduction of molecular oxygen to two molecules of water [GO:0016717]